regulation of ascospore-type prospore membrane formation [GO:1903023] (biological process) Relationships: is a type of GO:0010564; is a type of regulation of cellular component biogenesis [GO:0044087]; is_a GO:0050793; is a type of regulation of cellular component organization [GO:0051128]; is a type of regulation of reproductive process [GO:2000241]; regulates ascospore-type prospore membrane formation [GO:0032120] Subtypes: positive regulation of ascospore-type prospore membrane formation [GO:1903024] References: PMID:11405625 Sources: GOC:TermGenie, GO_REF:0000058 Definition: Any process that modulates the frequency, rate or extent of formation of an ascospore-type prospore membrane. Also known as: regulation of FSM assembly, regulation of FSM biosynthesis, regulation of FSM formation, regulation of forespore membrane biosynthesis, regulation of forespore membrane formation, regulation of ascospore-type prospore membrane assembly